{
  "term_label": "Unknown biological process",
  "gene_symbol": "SPANXA2-OT1",
  "gene_name": "Putative uncharacterized protein SPANXA2-OT1",
  "term_id": "UNKNOWN:0002",
  "gene": "UniProtKB:Q8N9U9"
}